sensory perception of wind [GO:0071063] (biological process) Definition: The series of events required for an organism to receive sensory mechanical stimulus resulting from air flow, convert it to a molecular signal, and recognize and characterize the signal. Also known as: perception of wind, sensory perception of air flow Relationships: is a type of GO:0050954 References: PMID:19279637 Sources: GOC:mah